{
  "term_label": "phototransduction",
  "term_id": "GO:0007602",
  "gene_symbol": "OPN5",
  "gene_name": "Opsin-5",
  "gene": "UniProtKB:Q6U736"
}